{
  "gene_name": "Homeobox protein Hox-B2",
  "gene": "UniProtKB:P14652",
  "gene_symbol": "HOXB2",
  "term_label": "regulation of transcription by RNA polymerase II",
  "term_id": "GO:0006357"
}